{
  "term_label": "Unknown cellular component",
  "term_id": "UNKNOWN:0003",
  "gene_symbol": "METTL17",
  "gene_name": "Methyltransferase-like protein 17, mitochondrial",
  "gene": "UniProtKB:Q9H7H0"
}